{
  "gene_name": "THO complex subunit 6 homolog",
  "gene": "UniProtKB:Q86W42",
  "term_id": "GO:0000347",
  "gene_symbol": "THOC6",
  "term_label": "THO complex"
}